{
  "term_id": "GO:0003735",
  "gene_symbol": "SRBD1",
  "gene_name": "S1 RNA-binding domain-containing protein 1",
  "term_label": "structural constituent of ribosome",
  "gene": "UniProtKB:Q8N5C6"
}